{
  "gene": "UniProtKB:Q96NA2",
  "term_label": "ciliary basal body",
  "term_id": "GO:0036064",
  "gene_name": "Rab-interacting lysosomal protein",
  "gene_symbol": "RILP"
}